{
  "gene": "UniProtKB:Q16549",
  "gene_symbol": "PCSK7",
  "term_label": "serine-type endopeptidase activity",
  "term_id": "GO:0004252",
  "gene_name": "Proprotein convertase subtilisin_kexin type 7"
}